nuclear membrane [GO:0031965] (cellular component) Sources: GOC:mah, GOC:pz Definition: Either of the lipid bilayers that surround the nucleus and form the nuclear envelope; excludes the intermembrane space. Subtypes: GO:0005637, nuclear outer membrane [GO:0005640] Relationships: is a type of organelle membrane [GO:0031090]; is part of nuclear envelope [GO:0005635]